{
  "term_label": "histone H3K4me/H3K4me2/H3K4me3 demethylase activity",
  "gene_name": "Lysine-specific demethylase 5A",
  "gene_symbol": "KDM5A",
  "term_id": "GO:0034647",
  "gene": "UniProtKB:P29375"
}